{
  "gene_name": "Ficolin-1",
  "gene": "UniProtKB:O00602",
  "term_label": "extracellular matrix",
  "term_id": "GO:0031012",
  "gene_symbol": "FCN1"
}